{
  "gene": "UniProtKB:Q92900",
  "gene_symbol": "UPF1",
  "gene_name": "Regulator of nonsense transcripts 1",
  "term_id": "GO:0000184",
  "term_label": "nuclear-transcribed mRNA catabolic process, nonsense-mediated decay"
}